{
  "gene": "UniProtKB:Q9NRY7",
  "gene_symbol": "PLSCR2",
  "term_id": "GO:0070782",
  "term_label": "phosphatidylserine exposure on apoptotic cell surface",
  "gene_name": "Phospholipid scramblase 2"
}